nucleoside monophosphate metabolic process [GO:0009123] (biological process) Also known as: nucleoside monophosphate metabolism Sources: GOC:go_curators, ISBN:0198506732 Subtypes: nucleoside monophosphate biosynthetic process [GO:0009124], nucleoside monophosphate catabolic process [GO:0009125], purine nucleoside monophosphate metabolic process [GO:0009126], pyrimidine nucleoside monophosphate metabolic process [GO:0009129], GO:0046444, nucleoside monophosphate phosphorylation [GO:0046940] Relationships: is a type of nucleoside phosphate metabolic process [GO:0006753] Definition: The chemical reactions and pathways involving a nucleoside monophosphate, a compound consisting of a nucleobase linked to a deoxyribose or ribose sugar esterified with phosphate on the sugar.